{
  "gene": "UniProtKB:O14494",
  "gene_name": "Phospholipid phosphatase 1",
  "gene_symbol": "PLPP1",
  "term_id": "GO:0007165",
  "term_label": "signal transduction"
}